{
  "term_label": "poly(A) RNA polymerase activity",
  "term_id": "GO:1990817",
  "gene": "UniProtKB:Q8NEK8",
  "gene_name": "Terminal nucleotidyltransferase 5D",
  "gene_symbol": "TENT5D"
}